protein deglutarylation [GO:0061698] (biological process) References: PMID:24703693 Sources: GOC:dph Definition: The removal of a glutaryl group (CO-CH2-CH2-CH2-CO) from a residue in a peptide or protein. Relationships: is a type of protein deacylation [GO:0035601]